positive regulation of early endosome to late endosome transport [GO:2000643] (biological process) Sources: GOC:BHF Relationships: is a type of positive regulation of intracellular transport [GO:0032388]; is a type of GO:2000641; positively regulates GO:0045022 Definition: Any process that activates or increases the frequency, rate or extent of early endosome to late endosome transport.